{
  "gene_name": "Caspase activity and apoptosis inhibitor 1",
  "gene": "UniProtKB:Q9H8G2",
  "term_id": "UNKNOWN:0003",
  "gene_symbol": "CAAP1",
  "term_label": "Unknown cellular component"
}